{
  "gene": "UniProtKB:O95859",
  "term_label": "Unknown biological process",
  "term_id": "UNKNOWN:0002",
  "gene_name": "Tetraspanin-12",
  "gene_symbol": "TSPAN12"
}